{
  "gene_name": "Melanocortin-2 receptor accessory protein",
  "term_id": "GO:0005783",
  "term_label": "endoplasmic reticulum",
  "gene": "UniProtKB:Q8TCY5",
  "gene_symbol": "MRAP"
}